{
  "term_label": "antimicrobial humoral immune response mediated by antimicrobial peptide",
  "gene": "UniProtKB:P55773",
  "gene_symbol": "CCL23",
  "gene_name": "C-C motif chemokine 23",
  "term_id": "GO:0061844"
}